{
  "gene_symbol": "GABRG2",
  "gene_name": "Gamma-aminobutyric acid receptor subunit gamma-2",
  "term_id": "GO:0022851",
  "gene": "UniProtKB:P18507",
  "term_label": "GABA-gated chloride ion channel activity"
}